{
  "gene": "UniProtKB:P56975",
  "term_label": "ERBB4 signaling pathway",
  "gene_name": "Pro-neuregulin-3, membrane-bound isoform",
  "gene_symbol": "NRG3",
  "term_id": "GO:0038130"
}